{
  "gene": "UniProtKB:E5RHQ5",
  "term_label": "Unknown biological process",
  "gene_name": "Nuclear pore complex-interacting protein family member B11",
  "term_id": "UNKNOWN:0002",
  "gene_symbol": "NPIPB11"
}